leukocyte apoptotic process [GO:0071887] (biological process) Note: Note that a lymphocyte is a cell of the B cell, T cell, or natural killer cell lineage (CL:0000542). Also known as: leukocyte apoptosis Relationships: is a type of GO:0006915 Sources: CL:0000738, GOC:BHF, GOC:mah, GOC:mtg_apoptosis Definition: Any apoptotic process in a leukocyte, an achromatic cell of the myeloid or lymphoid lineages capable of ameboid movement, found in blood or other tissue. Subtypes: neutrophil apoptotic process [GO:0001781], mast cell apoptotic process [GO:0033024], GO:0070227, macrophage apoptotic process [GO:0071888], dendritic cell apoptotic process [GO:0097048] Regulation: RO_0002211 by regulation of leukocyte apoptotic process [GO:2000106]; negatively regulated by negative regulation of leukocyte apoptotic process [GO:2000107]; positively regulated by positive regulation of leukocyte apoptotic process [GO:2000108]